{
  "gene_name": "Gamma-2-syntrophin",
  "term_id": "UNKNOWN:0002",
  "term_label": "Unknown biological process",
  "gene": "UniProtKB:Q9NY99",
  "gene_symbol": "SNTG2"
}